{
  "gene_name": "Protein Wnt-11",
  "gene": "UniProtKB:O96014",
  "term_id": "GO:0060070",
  "term_label": "canonical Wnt signaling pathway",
  "gene_symbol": "WNT11"
}